{
  "term_id": "GO:0060326",
  "term_label": "cell chemotaxis",
  "gene": "UniProtKB:Q9NPB9",
  "gene_symbol": "ACKR4",
  "gene_name": "Atypical chemokine receptor 4"
}